4-hydroxyphenylacetate 3-monooxygenase activity [GO:0052881] (MF) Definition: Catalysis of the reaction: (4-hydroxyphenyl)acetate + FADH(2) + O2 = 3,4-dihydroxyphenylacetate + FAD + H+ + H2O. Relationships: is a type of oxidoreductase activity, acting on paired donors, with incorporation or reduction of molecular oxygen, reduced flavin or flavoprotein as one donor, and incorporation of one atom of oxygen [GO:0016712] Also known as: 4 HPA 3-hydroxylase activity, 4-hydroxyphenylacetic acid-3-hydroxylase activity, p-hydroxyphenylacetate 3-hydroxylase activity, p-hydroxyphenylacetate hydroxylase activity, 4-hydroxyphenylacetate,FADH:oxygen oxidoreductase (3-hydroxylating) activity, p-hydroxyphenylacetate 3-hydroxylase (FAD) activity, p-hydroxyphenylacetate hydroxylase (FAD) activity Sources: RHEA:30595